{
  "gene_symbol": "MINAR1",
  "gene": "UniProtKB:Q9UPX6",
  "gene_name": "Major intrinsically disordered Notch2-binding receptor 1",
  "term_label": "negative regulation of cell population proliferation",
  "term_id": "GO:0008285"
}